fibroblast chemotaxis [GO:1990956] (biological process) Regulation: regulated by regulation of fibroblast chemotaxis [GO:1905210]; RO_0002212 by negative regulation of fibroblast chemotaxis [GO:1905211]; positively regulated by positive regulation of fibroblast chemotaxis [GO:1905212] References: PMID:8760137 Sources: GOC:dph Definition: The directed movement of a fibroblast guided by a specific chemical concentration gradient. Movement may be towards a higher concentration (positive chemotaxis) or towards a lower concentration (negative chemotaxis). Relationships: is a type of GO:0060326